(+)-sesaminol 2-O-glucosyltransferase activity [GO:0102423] (molecular function) Definition: Catalysis of the reaction: (+)-sesaminol + UDP-alpha-D-glucose = (+)-sesaminol 2-O-beta-D-glucoside + UDP + H+. Relationships: is a type of hexosyltransferase activity [GO:0016758] References: PMID:18248594, PMID:19561332 Sources: GOC:pz